{
  "gene": "UniProtKB:Q14258",
  "gene_name": "E3 ubiquitin_ISG15 ligase TRIM25",
  "gene_symbol": "TRIM25",
  "term_label": "Unknown molecular function",
  "term_id": "UNKNOWN:0001"
}